{
  "term_label": "positive regulation of amino acid transport",
  "gene_name": "Collectrin",
  "gene_symbol": "CLTRN",
  "term_id": "GO:0051957",
  "gene": "UniProtKB:Q9HBJ8"
}